{
  "term_id": "GO:0005886",
  "gene_symbol": "PLAUR",
  "term_label": "plasma membrane",
  "gene": "UniProtKB:Q03405",
  "gene_name": "Urokinase plasminogen activator surface receptor"
}